{
  "term_label": "cell surface",
  "gene": "UniProtKB:Q9BXN2",
  "gene_name": "C-type lectin domain family 7 member A",
  "term_id": "GO:0009986",
  "gene_symbol": "CLEC7A"
}